CD4-positive, alpha-beta T cell differentiation involved in immune response [GO:0002294] (biological process) Subtypes: GO:0002298, GO:0042093 Note: Note that immunologists typically use the word 'development' to refer to cells of B or T cell lineages undergoing the process that GO describes as 'cell differentiation'. Sources: GOC:add, ISBN:0781735149 Relationships: is a type of alpha-beta T cell differentiation involved in immune response [GO:0002293]; is_a GO:0043367 Also known as: CD4-positive, alpha-beta T cell development involved in immune response, CD4-positive, alpha-beta T cell differentiation during immune response, CD4-positive, alpha-beta T lymphocyte differentiation during immune response, CD4-positive, alpha-beta T-cell differentiation during immune response, CD4-positive, alpha-beta T-lymphocyte differentiation during immune response Definition: The process in which an antigenically naive CD4-positive, alpha-beta T cell acquires the specialized features of an effector, regulatory, or memory T cell as part of an immune response. Effector T cells include cells which provide T cell help or exhibit cytotoxicity towards other cells.